{
  "gene_symbol": "BSN",
  "term_label": "structural constituent of presynaptic active zone",
  "gene": "UniProtKB:Q9UPA5",
  "term_id": "GO:0098882",
  "gene_name": "Protein bassoon"
}